{
  "gene_name": "B box and SPRY domain-containing protein",
  "gene": "UniProtKB:Q5W0U4",
  "gene_symbol": "BSPRY",
  "term_id": "GO:0005737",
  "term_label": "cytoplasm"
}